{
  "term_label": "protein-lysine-acetyltransferase activity",
  "gene_symbol": "ESCO2",
  "term_id": "GO:0061733",
  "gene": "UniProtKB:Q56NI9",
  "gene_name": "N-acetyltransferase ESCO2"
}